{
  "term_label": "acetylcholine receptor activity",
  "term_id": "GO:0015464",
  "gene_name": "Neuronal acetylcholine receptor subunit beta-3",
  "gene_symbol": "CHRNB3",
  "gene": "UniProtKB:Q05901"
}